{
  "gene_name": "Aldo-keto reductase family 1 member B10",
  "gene": "UniProtKB:O60218",
  "gene_symbol": "AKR1B10",
  "term_label": "mitochondrion",
  "term_id": "GO:0005739"
}